{
  "gene_name": "Transmembrane protein 151B",
  "gene": "UniProtKB:Q8IW70",
  "term_label": "Unknown biological process",
  "gene_symbol": "TMEM151B",
  "term_id": "UNKNOWN:0002"
}